{
  "gene_name": "Keratin-associated protein 3-1",
  "term_label": "Unknown cellular component",
  "term_id": "UNKNOWN:0003",
  "gene_symbol": "KRTAP3-1",
  "gene": "UniProtKB:Q9BYR8"
}